granulysin production [GO:0036262] (biological process) Relationships: is a type of production of molecular mediator of immune response [GO:0002440] Sources: GOC:rv Definition: The appearance of granulysin due to biosynthesis or secretion following a cellular stimulus, resulting in an increase in its intracellular or extracellular levels. Note: Note that this term is in the subset of terms that should not be used for direct gene product annotation. Instead, select one of the 'regulation' children terms.